{
  "term_id": "GO:0042771",
  "term_label": "intrinsic apoptotic signaling pathway in response to DNA damage by p53 class mediator",
  "gene": "UniProtKB:Q9BVC6",
  "gene_name": "Transmembrane protein 109",
  "gene_symbol": "TMEM109"
}